{
  "gene": "UniProtKB:A0A1W2PQ72",
  "gene_name": "Myb_SANT-like DNA-binding domain-containing protein 7",
  "term_label": "Unknown cellular component",
  "gene_symbol": "MSANTD7",
  "term_id": "UNKNOWN:0003"
}